{
  "gene": "UniProtKB:Q8NFY9",
  "gene_name": "Kelch repeat and BTB domain-containing protein 8",
  "term_label": "Cul3-RING ubiquitin ligase complex",
  "term_id": "GO:0031463",
  "gene_symbol": "KBTBD8"
}